{
  "gene": "UniProtKB:Q9Y258",
  "gene_name": "C-C motif chemokine 26",
  "term_id": "GO:0070098",
  "gene_symbol": "CCL26",
  "term_label": "chemokine-mediated signaling pathway"
}